{
  "gene_symbol": "LINC00173",
  "gene_name": "Putative uncharacterized protein encoded by LINC00173",
  "gene": "UniProtKB:Q6ZV60",
  "term_id": "UNKNOWN:0001",
  "term_label": "Unknown molecular function"
}